{
  "term_label": "membrane protein proteolysis",
  "gene": "UniProtKB:Q8TCT9",
  "gene_name": "Minor histocompatibility antigen H13",
  "gene_symbol": "HM13",
  "term_id": "GO:0033619"
}